{
  "term_label": "Unknown molecular function",
  "term_id": "UNKNOWN:0001",
  "gene": "UniProtKB:A0A075B6Y0",
  "gene_name": "T cell receptor alpha joining 49 (Fragment)",
  "gene_symbol": "TRAJ49"
}